maturation of 5S rRNA [GO:0000481] (biological process) Relationships: is a type of rRNA processing [GO:0006364] Definition: Any process involved in the maturation of a precursor 5S ribosomal RNA (rRNA) molecule into a mature 5S rRNA molecule. Sources: GOC:curators Subtypes: maturation of 5S rRNA from tetracistronic rRNA transcript (SSU-rRNA, 5.8S rRNA, LSU-rRNA) [GO:0000482], generation of mature 3'-end of 5S rRNA generated by RNA polymerase III [GO:0002107]